voltage-gated calcium channel complex [GO:0005891] (cellular component) Also known as: voltage gated calcium channel complex, voltage-dependent calcium channel complex, voltage-sensitive calcium channel complex Relationships: is a type of calcium channel complex [GO:0034704]; is a type of plasma membrane protein complex [GO:0098797] Definition: A protein complex that forms a transmembrane channel through which calcium ions may pass in response to changes in membrane potential. Sources: GOC:mah Subtypes: light-activated voltage-gated calcium channel complex [GO:0008087], CatSper complex [GO:0036128], GO:1990425, L-type voltage-gated calcium channel complex [GO:1990454]